tRNA (5-carboxymethyluridine(34)-5-O)-methyltransferase activity [GO:0106335] (molecular function) References: PMID:20123966 Sources: RHEA:43208 Relationships: is a type of tRNA (uridine) methyltransferase activity [GO:0016300] Definition: Catalysis of the reaction: 5-(carboxymethyl)uridine34 in tRNA + S-adenosyl-L-methionine = 5-(2-methoxy-2-oxoethyl)uridine34 in tRNA + S-adenosyl-L-homocysteine.